meiosis I spindle assembly checkpoint signaling [GO:1905318] (biological process) Relationships: is a type of meiotic spindle assembly checkpoint signaling [GO:0033316]; is a type of negative regulation of meiosis I [GO:0110029] Also known as: meiosis I spindle assembly checkpoint Definition: Any spindle assembly checkpoint that is involved in meiosis I. References: PMID:26483559 Sources: GOC:TermGenie, GO_REF:0000060 Regulation: regulated by regulation of meiosis I spindle assembly checkpoint [GO:1905325]; positively regulated by positive regulation of meiosis I spindle assembly checkpoint [GO:1905326]